{
  "term_id": "UNKNOWN:0001",
  "gene": "UniProtKB:Q8WUD4",
  "gene_name": "Coiled-coil domain-containing protein 12",
  "term_label": "Unknown molecular function",
  "gene_symbol": "CCDC12"
}